{
  "term_id": "GO:0030672",
  "gene": "UniProtKB:Q8TBG9",
  "gene_symbol": "SYNPR",
  "gene_name": "Synaptoporin",
  "term_label": "synaptic vesicle membrane"
}